{
  "term_label": "phosphatidylinositol dephosphorylation",
  "gene_name": "Myotubularin-related protein 9",
  "gene": "UniProtKB:Q96QG7",
  "gene_symbol": "MTMR9",
  "term_id": "GO:0046856"
}